{
  "term_label": "serine-tRNA ligase activity",
  "gene_name": "Serine--tRNA ligase, mitochondrial",
  "gene": "UniProtKB:Q9NP81",
  "gene_symbol": "SARS2",
  "term_id": "GO:0004828"
}